sperm capacitation [GO:0048240] (biological process) Note: Avian spermatozoa do not require a period of capacitation, since they are competent to fertilize the egg without a prolonged sojourn in the oviduct or in a capacitation medium in vitro. Therefore, sperm capacitation can only be applied to Aves to refer to gene products involved in processes that occur prior to sperm being deposited from the avian male. The term cannot apply to processes occurring in the avian female reproductive tract. Regulation: regulated by regulation of sperm capacitation [GO:1902490]; negatively regulated by negative regulation of sperm capacitation [GO:1902491]; positively regulated by positive regulation of sperm capacitation [GO:1902492] Definition: A process required for sperm to reach fertilization competence. Sperm undergo an incompletely understood series of morphological and molecular maturational processes, termed capacitation, involving, among other processes, protein tyrosine phosphorylation and increased intracellular calcium. Relationships: is a type of developmental process involved in reproduction [GO:0003006]; is_a GO:0022412; is_a GO:0048469; is part of spermatid development [GO:0007286] References: PMID:11820818 Sources: GOC:jid, ISBN:978-3-642-58301-8 Also known as: sperm activation